{
  "term_id": "UNKNOWN:0002",
  "gene": "UniProtKB:Q1RN00",
  "term_label": "Unknown biological process",
  "gene_name": "Putative uncharacterized protein LOC151760",
  "gene_symbol": "Q1RN00"
}